{
  "term_id": "GO:0005634",
  "gene_name": "Protein odd-skipped-related 2",
  "gene": "UniProtKB:Q8N2R0",
  "term_label": "nucleus",
  "gene_symbol": "OSR2"
}